{
  "term_label": "cell adhesion",
  "term_id": "GO:0007155",
  "gene_name": "Basal cell adhesion molecule",
  "gene": "UniProtKB:P50895",
  "gene_symbol": "BCAM"
}